{
  "gene_name": "Synaptotagmin-4",
  "term_id": "GO:0099502",
  "gene_symbol": "SYT4",
  "gene": "UniProtKB:Q9H2B2",
  "term_label": "calcium-dependent activation of synaptic vesicle fusion"
}